{
  "term_label": "positive regulation of stress fiber assembly",
  "term_id": "GO:0051496",
  "gene": "UniProtKB:Q15569",
  "gene_name": "Dual specificity testis-specific protein kinase 1",
  "gene_symbol": "TESK1"
}